{
  "gene": "UniProtKB:Q6NTF9",
  "term_id": "GO:0030968",
  "term_label": "endoplasmic reticulum unfolded protein response",
  "gene_name": "Rhomboid domain-containing protein 2",
  "gene_symbol": "RHBDD2"
}